{
  "gene_symbol": "SLC10A4",
  "term_id": "UNKNOWN:0001",
  "term_label": "Unknown molecular function",
  "gene_name": "Sodium_bile acid cotransporter 4",
  "gene": "UniProtKB:Q96EP9"
}